{
  "term_label": "cytosol",
  "gene_symbol": "DPYSL5",
  "gene_name": "Dihydropyrimidinase-related protein 5",
  "gene": "UniProtKB:Q9BPU6",
  "term_id": "GO:0005829"
}